{
  "term_id": "GO:0004984",
  "gene_symbol": "OR2A14",
  "term_label": "olfactory receptor activity",
  "gene_name": "Olfactory receptor 2A14",
  "gene": "UniProtKB:Q96R47"
}